{
  "term_id": "GO:0007268",
  "term_label": "chemical synaptic transmission",
  "gene_name": "Synaptotagmin-3",
  "gene": "UniProtKB:Q9BQG1",
  "gene_symbol": "SYT3"
}